{
  "gene_name": "Serine_threonine-protein kinase SMG1",
  "gene_symbol": "SMG1",
  "gene": "UniProtKB:Q96Q15",
  "term_id": "GO:0000184",
  "term_label": "nuclear-transcribed mRNA catabolic process, nonsense-mediated decay"
}